T-tubule organization [GO:0033292] (biological process) Definition: A process that is carried out at the cellular level that results in the assembly, arrangement of constituent parts, or disassembly of the T-tubule. A T-tubule is an invagination of the plasma membrane of a muscle cell that extends inward from the cell surface around each myofibril. Also known as: T-tubule organisation, transverse tubule organization, T-tubule organization and biogenesis Relationships: is_a membrane organization [GO:0061024]; is part of plasma membrane organization [GO:0007009]; BFO_0000050 muscle cell development [GO:0055001] Sources: GOC:dph, GOC:jl, GOC:mah